histone serotonyltransferase activity [GO:0120295] (molecular function) Definition: Catalysis of the reaction: L-glutaminyl-[histone] + serotonin = 5-serotonyl-L-glutamyl-[histone] + NH4(+). References: PMID:30867594 Sources: GOC:sp Relationships: is a type of peptide serotonyltransferase activity [GO:0120294]; is a type of histone modifying activity [GO:0140993]